{
  "term_id": "GO:0051537",
  "gene_name": "Iron-sulfur cluster assembly enzyme ISCU",
  "gene_symbol": "ISCU",
  "gene": "UniProtKB:Q9H1K1",
  "term_label": "2 iron, 2 sulfur cluster binding"
}